{
  "gene_symbol": "LY75",
  "gene": "UniProtKB:O60449",
  "gene_name": "Lymphocyte antigen 75",
  "term_label": "transmembrane signaling receptor activity",
  "term_id": "GO:0004888"
}